{
  "term_label": "Unknown cellular component",
  "gene": "UniProtKB:Q13573",
  "term_id": "UNKNOWN:0003",
  "gene_symbol": "SNW1",
  "gene_name": "SNW domain-containing protein 1"
}